{
  "gene": "UniProtKB:P61586",
  "gene_name": "Transforming protein RhoA",
  "term_id": "GO:0003924",
  "term_label": "GTPase activity",
  "gene_symbol": "RHOA"
}